{
  "term_id": "GO:0007423",
  "gene_name": "Neurogenic differentiation factor 6",
  "term_label": "sensory organ development",
  "gene": "UniProtKB:Q96NK8",
  "gene_symbol": "NEUROD6"
}